{
  "term_id": "UNKNOWN:0002",
  "gene": "UniProtKB:P00387",
  "gene_symbol": "CYB5R3",
  "gene_name": "NADH-cytochrome b5 reductase 3",
  "term_label": "Unknown biological process"
}